{
  "gene_name": "Cerebral dopamine neurotrophic factor",
  "term_id": "GO:0071542",
  "term_label": "dopaminergic neuron differentiation",
  "gene_symbol": "CDNF",
  "gene": "UniProtKB:Q49AH0"
}